{
  "gene_symbol": "TFAP2C",
  "gene": "UniProtKB:Q92754",
  "term_label": "nucleus",
  "gene_name": "Transcription factor AP-2 gamma",
  "term_id": "GO:0005634"
}